regulation of mesenchymal cell apoptotic process involved in nephron morphogenesis [GO:0072039] (BP) Subtypes: regulation of mesenchymal cell apoptotic process involved in mesonephric nephron morphogenesis [GO:0061295], negative regulation of mesenchymal cell apoptotic process involved in nephron morphogenesis [GO:0072040], positive regulation of mesenchymal cell apoptotic process involved in nephron morphogenesis [GO:0072041], regulation of mesenchymal cell apoptotic process involved in metanephric nephron morphogenesis [GO:0072304] Definition: Any process that modulates the occurrence or rate of mesenchymal stem cell death by apoptotic process that contributes to the shaping of the nephron. Relationships: is a type of GO:1902337; is a type of regulation of somatic stem cell population maintenance [GO:1904672]; is a type of regulation of mesenchymal cell apoptotic process [GO:2001053]; regulates mesenchymal stem cell maintenance involved in nephron morphogenesis [GO:0072038]; regulates mesenchymal cell apoptotic process involved in nephron morphogenesis [GO:1901145] Also known as: regulation of mesenchymal stem cell apoptotic process involved in nephron morphogenesis, regulation of mesenchymal stem cell apoptosis involved in nephron morphogenesis Sources: GOC:mtg_apoptosis, GOC:mtg_kidney_jan10